{
  "gene_symbol": "DPP7",
  "term_label": "vesicle",
  "term_id": "GO:0031982",
  "gene_name": "Dipeptidyl peptidase 2",
  "gene": "UniProtKB:Q9UHL4"
}